K antigen metabolic process [GO:0046375] (biological process) Subtypes: GO:0009248 Definition: The chemical reactions and pathways involving K antigen, a capsular polysaccharide antigen carried on the surface of bacterial capsules that masks somatic (O) antigens. Also known as: K antigen metabolism Relationships: is a type of GO:0043170; is a type of carbohydrate derivative metabolic process [GO:1901135] Sources: ISBN:0198506732